{
  "term_id": "UNKNOWN:0001",
  "gene": "UniProtKB:Q76KD6",
  "term_label": "Unknown molecular function",
  "gene_name": "Speriolin",
  "gene_symbol": "SPATC1"
}